{
  "gene_symbol": "ACAA1",
  "gene_name": "3-ketoacyl-CoA thiolase, peroxisomal",
  "term_id": "GO:0010124",
  "gene": "UniProtKB:P09110",
  "term_label": "phenylacetate catabolic process"
}